{
  "gene": "UniProtKB:O43593",
  "gene_name": "Lysine-specific demethylase hairless",
  "gene_symbol": "HR",
  "term_label": "chromatin",
  "term_id": "GO:0000785"
}